{
  "gene_symbol": "SMARCB1",
  "term_label": "chromatin remodeling",
  "gene": "UniProtKB:Q12824",
  "term_id": "GO:0006338",
  "gene_name": "SWI_SNF-related matrix-associated actin-dependent regulator of chromatin subfamily B member 1"
}